{
  "gene_symbol": "ZC3H7A",
  "term_id": "UNKNOWN:0003",
  "term_label": "Unknown cellular component",
  "gene_name": "Zinc finger CCCH domain-containing protein 7A",
  "gene": "UniProtKB:Q8IWR0"
}